{
  "gene": "UniProtKB:Q969H9",
  "term_label": "Unknown biological process",
  "term_id": "UNKNOWN:0002",
  "gene_name": "Disrupted in renal carcinoma protein 1",
  "gene_symbol": "DIRC1"
}